tRNA-specific adenosine-37 deaminase activity [GO:0043829] (molecular function) Also known as: tRNA(Ala)-A37 deaminase activity, tRNA-specific adenosine deaminase 1, TAD1 Definition: Catalysis of the reaction: adenosine-37 + H2O = inosine-37 + NH3, in a tRNA-Ala molecule. Relationships: is a type of GO:0008251 References: PMID:8915538, PMID:9707437 Sources: RHEA:50968